{
  "gene_symbol": "SLC1A6",
  "gene_name": "Excitatory amino acid transporter 4",
  "term_label": "L-glutamate transmembrane transporter activity",
  "term_id": "GO:0005313",
  "gene": "UniProtKB:P48664"
}